{
  "gene_symbol": "ARHGEF2",
  "term_label": "guanyl-nucleotide exchange factor activity",
  "gene_name": "Rho guanine nucleotide exchange factor 2",
  "gene": "UniProtKB:Q92974",
  "term_id": "GO:0005085"
}